{
  "gene": "UniProtKB:C9JE40",
  "term_id": "GO:0003723",
  "term_label": "RNA binding",
  "gene_symbol": "PATL2",
  "gene_name": "Protein PAT1 homolog 2"
}